{
  "term_label": "mitochondrion",
  "gene": "UniProtKB:P16219",
  "gene_symbol": "ACADS",
  "term_id": "GO:0005739",
  "gene_name": "Short-chain specific acyl-CoA dehydrogenase, mitochondrial"
}